{
  "gene_name": "Putative tyrosine-protein phosphatase auxilin",
  "term_id": "GO:0014069",
  "term_label": "postsynaptic density",
  "gene_symbol": "DNAJC6",
  "gene": "UniProtKB:O75061"
}